{
  "gene_name": "Kinesin-like protein KIF18A",
  "term_label": "nucleus",
  "gene": "UniProtKB:Q8NI77",
  "term_id": "GO:0005634",
  "gene_symbol": "KIF18A"
}